{
  "gene_name": "D(2) dopamine receptor",
  "gene": "UniProtKB:P14416",
  "term_label": "regulation of dopamine secretion",
  "gene_symbol": "DRD2",
  "term_id": "GO:0014059"
}